purine nucleoside diphosphate metabolic process [GO:0009135] (biological process) Definition: The chemical reactions and pathways involving purine nucleoside diphosphate, a compound consisting of a purine base linked to a ribose or deoxyribose sugar esterified with diphosphate on the sugar. Sources: GOC:go_curators, ISBN:0198506732 Also known as: purine nucleoside diphosphate metabolism Relationships: is a type of nucleoside diphosphate metabolic process [GO:0009132] Subtypes: GO:0009136, purine nucleoside diphosphate catabolic process [GO:0009137], purine ribonucleoside diphosphate metabolic process [GO:0009179], purine deoxyribonucleoside diphosphate metabolic process [GO:0009182]